regulation of amino acid biosynthetic process [GO:2000282] (biological process) Relationships: is a type of regulation of amino acid metabolic process [GO:0006521]; is a type of regulation of biosynthetic process [GO:0009889]; regulates GO:0008652 Also known as: regulation of cellular amino acid anabolism, regulation of cellular amino acid biosynthesis, regulation of cellular amino acid biosynthetic process, regulation of cellular amino acid formation, regulation of cellular amino acid synthesis Sources: GOC:obol Definition: Any process that modulates the frequency, rate or extent of cellular amino acid biosynthetic process. Subtypes: regulation of L-glutamine biosynthetic process [GO:0062132], regulation of histidine biosynthetic process [GO:0120213], GO:1900079, regulation of homoserine biosynthetic process [GO:1901710], regulation of L-proline biosynthetic process [GO:1902005], regulation of lysine biosynthetic process via aminoadipic acid [GO:1902986], regulation of L-dopa biosynthetic process [GO:1903195], regulation of citrulline biosynthetic process [GO:1903248], negative regulation of amino acid biosynthetic process [GO:2000283], positive regulation of amino acid biosynthetic process [GO:2000284], GO:2001276